formation of cytoplasmic translation initiation complex [GO:0001732] (biological process) Definition: Joining of the large ribosomal subunit with the translation preinitiation complex, with release of IF2/eIF2 and IF3/eIF3 or IF5B/eIF5B. This leaves the functional ribosome at the AUG, with the methionyl/formyl-methionyl-tRNA positioned at the P site. References: PMID:29735639 Sources: GOC:hjd Also known as: formation of translation initiation complex, translation initiation complex assembly, cytoplasmic translation initiation complex assembly Relationships: is a type of GO:0022618; is part of cytoplasmic translational initiation [GO:0002183]